EGFR-Shc-Grb2-Sos complex [GO:0070621] (cellular component) Definition: A protein complex that contains the epidermal growth factor receptor (EGFR), Grb2, the adaptor protein SHC and the guanine nucleotide exchange factor Sos (or an ortholog thereof, such as mSos1), and is involved in linking EGFR activation to the p21-Ras pathway. References: PMID:7798267, PMID:8940013 Sources: GOC:mah Relationships: is a type of GO:0098797